{
  "gene": "UniProtKB:A6NN06",
  "term_label": "Unknown cellular component",
  "term_id": "UNKNOWN:0003",
  "gene_symbol": "A6NN06",
  "gene_name": "Putative UPF0633 protein MGC21881"
}